{
  "gene_symbol": "KIF28P",
  "gene": "UniProtKB:B7ZC32",
  "term_id": "GO:0008017",
  "term_label": "microtubule binding",
  "gene_name": "Kinesin-like protein KIF28P"
}